neural precursor cell proliferation [GO:0061351] (biological process) Sources: GOC:dph, GOC:yaf Definition: The multiplication or reproduction of neural precursor cells, resulting in the expansion of a cell population. A neural precursor cell is either a nervous system stem cell or a nervous system progenitor cell. Subtypes: neuroblast proliferation [GO:0007405], cell proliferation in dorsal spinal cord [GO:0010456], GO:0021534, cell proliferation in forebrain [GO:0021846], cell proliferation involved in neural plate elongation [GO:0021992], rhombomere cell proliferation [GO:0022034], GO:0033278, GO:0070444 Relationships: is a type of cell population proliferation [GO:0008283] Regulation: regulated by GO:2000177; negatively regulated by negative regulation of neural precursor cell proliferation [GO:2000178]; RO_0002213 by GO:2000179